peptidyl-serine autophosphorylation [GO:0036289] (biological process) Relationships: is a type of peptidyl-serine phosphorylation [GO:0018105]; is a type of protein autophosphorylation [GO:0046777] Also known as: serine autophosphorylation Subtypes: peptidyl-serine trans-autophosphorylation [GO:1990579] Sources: GOC:pm Definition: The phosphorylation by a protein of one or more of its own serine amino acid residues, or a serine residue on an identical protein.